{
  "term_label": "co-receptor binding",
  "gene_symbol": "DKK4",
  "gene_name": "Dickkopf-related protein 4",
  "term_id": "GO:0039706",
  "gene": "UniProtKB:Q9UBT3"
}